{
  "term_id": "GO:0008017",
  "gene_name": "Dynamin-1",
  "gene": "UniProtKB:Q05193",
  "gene_symbol": "DNM1",
  "term_label": "microtubule binding"
}